{
  "term_label": "piecemeal microautophagy of the nucleus",
  "gene_name": "Sorting nexin-7",
  "gene": "UniProtKB:Q9UNH6",
  "term_id": "GO:0034727",
  "gene_symbol": "SNX7"
}